{
  "term_label": "extracellular matrix",
  "gene_name": "Fibrinogen C domain-containing protein 1",
  "gene": "UniProtKB:Q8N539",
  "gene_symbol": "FIBCD1",
  "term_id": "GO:0031012"
}